aspartate:glutamate, proton antiporter activity [GO:0000515] (molecular function) Also known as: aspartate:glutamate antiporter activity References: PMID:11566871 Sources: RHEA:70783 Definition: Enables the transfer of a solute or solutes from one side of a membrane to the other according to the reaction: H+(out) + L-aspartate(in) + L-glutamate(out) = H+(in) + L-aspartate(out) + L-glutamate(in). Relationships: is_a L-aspartate transmembrane transporter activity [GO:0015183]; is a type of L-glutamate:proton antiporter activity [GO:0106421]